negative regulation of dauer entry [GO:1905910] (biological process) Definition: Any process that stops, prevents or reduces the frequency, rate or extent of dauer entry. References: PMID:21531333 Sources: GOC:TermGenie, GO_REF:0000058 Also known as: down regulation of dauer entry, down regulation of nematode entry into dormancy, down-regulation of dauer entry, down-regulation of nematode entry into dormancy, downregulation of dauer entry, downregulation of nematode entry into dormancy, negative regulation of nematode entry into dormancy, inhibition of dauer entry, inhibition of nematode entry into dormancy Relationships: is a type of negative regulation of dauer larval development [GO:0061067]; is a type of regulation of dauer entry [GO:1905909]; negatively regulates GO:0043053